{
  "term_id": "GO:0016581",
  "term_label": "NuRD complex",
  "gene_name": "Histone-binding protein RBBP4",
  "gene_symbol": "RBBP4",
  "gene": "UniProtKB:Q09028"
}